{
  "gene": "UniProtKB:Q8NET1",
  "term_id": "UNKNOWN:0003",
  "gene_name": "Beta-defensin 108B",
  "term_label": "Unknown cellular component",
  "gene_symbol": "DEFB108B"
}